positive regulation of blood coagulation [GO:0030194] (biological process) Definition: Any process that activates or increases the frequency, rate or extent of blood coagulation. Also known as: up regulation of blood coagulation, up-regulation of blood coagulation, upregulation of blood coagulation, activation of blood coagulation, stimulation of blood coagulation Relationships: is_a GO:0030193; is a type of GO:0050820; is a type of positive regulation of wound healing [GO:0090303]; is a type of positive regulation of hemostasis [GO:1900048]; positively regulates blood coagulation [GO:0007596] Sources: GOC:mah Subtypes: activation of blood coagulation via clotting cascade [GO:0002543], negative regulation of fibrinolysis [GO:0051918], GO:0097045, GO:2000262, positive regulation of blood coagulation, extrinsic pathway [GO:2000265], positive regulation of blood coagulation, intrinsic pathway [GO:2000268]